{
  "gene_name": "Transcription factor-like 5 protein",
  "gene": "UniProtKB:Q9UL49",
  "gene_symbol": "TCFL5",
  "term_label": "DNA-binding transcription factor activity, RNA polymerase II-specific",
  "term_id": "GO:0000981"
}